{
  "term_label": "antiviral innate immune response",
  "gene_symbol": "OASL",
  "term_id": "GO:0140374",
  "gene": "UniProtKB:Q15646",
  "gene_name": "2'-5'-oligoadenylate synthase-like protein"
}